{
  "term_id": "GO:0005737",
  "gene_symbol": "RNF130",
  "term_label": "cytoplasm",
  "gene": "UniProtKB:Q86XS8",
  "gene_name": "E3 ubiquitin-protein ligase RNF130"
}